vitamin catabolic process [GO:0009111] (biological process) Sources: GOC:ai Subtypes: fat-soluble vitamin catabolic process [GO:0042363], GO:0042365 Also known as: vitamin breakdown, vitamin catabolism, vitamin degradation Definition: The chemical reactions and pathways resulting in the breakdown of a vitamin, one of a number of unrelated organic substances that occur in many foods in small amounts and that are necessary in trace amounts for the normal metabolic functioning of the body, carried out by individual cells. Relationships: is_a vitamin metabolic process [GO:0006766]; is a type of small molecule catabolic process [GO:0044282]